{
  "term_label": "neurotransmitter loading into synaptic vesicle",
  "gene_symbol": "SLC32A1",
  "gene_name": "Vesicular inhibitory amino acid transporter",
  "term_id": "GO:0098700",
  "gene": "UniProtKB:Q9H598"
}